{
  "gene_symbol": "KIF22",
  "gene": "UniProtKB:Q14807",
  "term_label": "microtubule",
  "gene_name": "Kinesin-like protein KIF22",
  "term_id": "GO:0005874"
}